{
  "gene_symbol": "ABCB6",
  "term_label": "transmembrane transport",
  "gene": "UniProtKB:Q9NP58",
  "term_id": "GO:0055085",
  "gene_name": "ATP-binding cassette sub-family B member 6"
}